{
  "term_id": "GO:0005737",
  "term_label": "cytoplasm",
  "gene_symbol": "GCHFR",
  "gene_name": "GTP cyclohydrolase 1 feedback regulatory protein",
  "gene": "UniProtKB:P30047"
}